{
  "term_label": "oligosaccharide biosynthetic process",
  "term_id": "GO:0009312",
  "gene_name": "Mannose-P-dolichol utilization defect 1 protein",
  "gene_symbol": "MPDU1",
  "gene": "UniProtKB:O75352"
}